2-oxopropyl-CoM reductase (carboxylating) activity [GO:0050628] (molecular function) Definition: Catalysis of the reaction: acetoacetate + coenzyme M + NADP+ = 2-oxopropyl-coenzyme M + CO2 + NADPH. Sources: EC:1.8.1.5, RHEA:16977 Relationships: is a type of oxidoreductase activity, acting on a sulfur group of donors, NAD(P) as acceptor [GO:0016668] Also known as: 2-KPCC activity, 2-mercaptoethanesulfonate,acetoacetate:NADP+ oxidoreductase (decarboxylating), NADPH:2-(2-ketopropylthio)ethanesulfonate oxidoreductase/carboxylase activity, NADPH:2-ketopropyl-coenzyme M oxidoreductase/carboxylase activity